{
  "gene": "UniProtKB:Q96QK8",
  "term_id": "GO:0005783",
  "term_label": "endoplasmic reticulum",
  "gene_symbol": "SMIM14",
  "gene_name": "Small integral membrane protein 14"
}